{
  "gene_name": "1-phosphatidylinositol 4,5-bisphosphate phosphodiesterase beta-3",
  "gene": "UniProtKB:Q01970",
  "gene_symbol": "PLCB3",
  "term_id": "GO:0046488",
  "term_label": "phosphatidylinositol metabolic process"
}